{
  "gene": "UniProtKB:P13010",
  "gene_symbol": "XRCC5",
  "gene_name": "X-ray repair cross-complementing protein 5",
  "term_id": "GO:0000723",
  "term_label": "telomere maintenance"
}